{
  "gene_symbol": "RIC8B",
  "term_label": "G protein-coupled receptor signaling pathway",
  "gene": "UniProtKB:Q9NVN3",
  "gene_name": "Synembryn-B",
  "term_id": "GO:0007186"
}